{
  "term_label": "nuclear speck",
  "gene": "UniProtKB:Q5T200",
  "term_id": "GO:0016607",
  "gene_name": "Zinc finger CCCH domain-containing protein 13",
  "gene_symbol": "ZC3H13"
}